procollagen-proline 3-dioxygenase activity [GO:0019797] (molecular function) Sources: EC:1.14.11.7, RHEA:22872 Relationships: is a type of GO:0019798; is a type of peptidyl-proline 3-dioxygenase activity [GO:0031544] Also known as: prolyl 3-hydroxylase activity, procollagen-L-proline,2-oxoglutarate:oxygen oxidoreductase (3-hydroxylating) activity, procollagen-proline,2-oxoglutarate 3-dioxygenase activity, proline,2-oxoglutarate 3-dioxygenase activity, prolyl-4-hydroxyprolyl-glycyl-peptide, 2-oxoglutarate: oxygen oxidoreductase, 3-hydroxylating activity, protocollagen proline 3-hydroxylase activity Definition: Catalysis of the reaction: procollagen L-proline + 2-oxoglutarate + O2 = procollagen trans-3-hydroxy-L-proline + succinate + CO2.